{
  "term_id": "GO:0019901",
  "gene": "UniProtKB:P60953",
  "gene_name": "Cell division control protein 42 homolog",
  "gene_symbol": "CDC42",
  "term_label": "protein kinase binding"
}